positive regulation of immune response [GO:0050778] (biological process) Sources: GOC:ai Definition: Any process that activates or increases the frequency, rate or extent of the immune response, the immunological reaction of an organism to an immunogenic stimulus. Subtypes: activation of immune response [GO:0002253], GO:0002821, GO:0002830, positive regulation of immune response to tumor cell [GO:0002839], positive regulation of inflammatory response to antigenic stimulus [GO:0002863], positive regulation of humoral immune response [GO:0002922], GO:0032828, positive regulation of CD4-positive, CD25-positive, alpha-beta regulatory T cell differentiation involved in immune response [GO:0032834], positive regulation of mast cell activation involved in immune response [GO:0033008], positive regulation of eosinophil degranulation [GO:0043311], GO:0043315, positive regulation of memory T cell differentiation [GO:0043382], positive regulation of innate immune response [GO:0045089], positive regulation of T-helper cell differentiation [GO:0045624], GO:0050857, positive regulation of Fc receptor mediated stimulatory signaling pathway [GO:0060369], positive regulation of plasma cell differentiation [GO:1900100], positive regulation of basophil degranulation [GO:1903583], positive regulation of T cell activation via T cell receptor contact with antigen bound to MHC molecule on antigen presenting cell [GO:2001190], positive regulation of gamma-delta T cell activation involved in immune response [GO:2001193] Also known as: up regulation of immune response, up-regulation of immune response, upregulation of immune response, stimulation of immune response Relationships: is a type of GO:0002684; is a type of positive regulation of response to stimulus [GO:0048584]; is a type of regulation of immune response [GO:0050776]; positively regulates GO:0006955